positive regulation of fibroblast growth factor production [GO:0090271] (BP) Relationships: is a type of positive regulation of cytokine production [GO:0001819]; is a type of regulation of fibroblast growth factor production [GO:0090270]; positively regulates fibroblast growth factor production [GO:0090269] Sources: GOC:BHF Definition: Any process that increases the rate, frequency or extent of the appearance of a fibroblast growth factor due to biosynthesis or secretion following a cellular stimulus, resulting in an increase in its intracellular or extracellular levels.